benzylsuccinate synthase activity [GO:0018805] (molecular function) Relationships: is a type of carbon-carbon lyase activity [GO:0016830] Sources: EC:4.1.99.11, RHEA:10416 Definition: Catalysis of the reaction: fumarate + toluene = 2-benzylsuccinate. Also known as: benzylsuccinate fumarate-lyase (toluene-forming), benzylsuccinate fumarate-lyase activity